{
  "term_label": "antigen binding",
  "gene_name": "Immunoglobulin heavy variable 3-53",
  "gene_symbol": "IGHV3-53",
  "term_id": "GO:0003823",
  "gene": "UniProtKB:P01767"
}